{
  "term_id": "GO:0030169",
  "gene_symbol": "MSR1",
  "term_label": "low-density lipoprotein particle binding",
  "gene": "UniProtKB:P21757",
  "gene_name": "Macrophage scavenger receptor types I and II"
}